{
  "gene_name": "PACRG-like protein",
  "gene": "UniProtKB:Q8N7B6",
  "term_id": "UNKNOWN:0003",
  "term_label": "Unknown cellular component",
  "gene_symbol": "PACRGL"
}